intermediate filament binding [GO:0019215] (MF) Definition: Binding to an intermediate filament, a distinct elongated structure, characteristically 10 nm in diameter, that occurs in the cytoplasm of higher eukaryotic cells. Intermediate filaments form a fibrous system, composed of chemically heterogeneous subunits and involved in mechanically integrating the various components of the cytoplasmic space. Relationships: is a type of binding [GO:0005488] Sources: ISBN:0198506732 Subtypes: GO:1990254